{
  "gene_name": "116 kDa U5 small nuclear ribonucleoprotein component",
  "term_label": "mRNA splicing, via spliceosome",
  "gene_symbol": "EFTUD2",
  "term_id": "GO:0000398",
  "gene": "UniProtKB:Q15029"
}